{
  "gene": "UniProtKB:Q8N427",
  "gene_symbol": "NME8",
  "gene_name": "Thioredoxin domain-containing protein 3",
  "term_label": "axoneme",
  "term_id": "GO:0005930"
}